{
  "term_label": "voltage-gated potassium channel complex",
  "gene_name": "Potassium voltage-gated channel subfamily E member 2",
  "term_id": "GO:0008076",
  "gene_symbol": "KCNE2",
  "gene": "UniProtKB:Q9Y6J6"
}